iron-sulfur transferase activity [GO:0036455] (molecular function) Definition: Catalysis of the transfer of a iron-sulfur cluster from one compound (donor) to another (acceptor). Sources: GOC:bhm Also known as: Fe-S transferase activity Relationships: is a type of transferase activity, transferring sulphur-containing groups [GO:0016782]